{
  "gene_symbol": "NARF",
  "gene_name": "Nuclear prelamin A recognition factor",
  "gene": "UniProtKB:Q9UHQ1",
  "term_label": "lamin binding",
  "term_id": "GO:0005521"
}